{
  "term_label": "protein kinase binding",
  "gene_symbol": "SPDYE16",
  "gene": "UniProtKB:A6NNV3",
  "term_id": "GO:0019901",
  "gene_name": "Putative speedy protein E16"
}